{
  "term_id": "GO:0006355",
  "gene_symbol": "SCRT2",
  "term_label": "regulation of DNA-templated transcription",
  "gene": "UniProtKB:Q9NQ03",
  "gene_name": "Transcriptional repressor scratch 2"
}